{
  "gene": "UniProtKB:P25063",
  "term_label": "regulation of cell-cell adhesion",
  "term_id": "GO:0022407",
  "gene_symbol": "CD24",
  "gene_name": "Signal transducer CD24"
}